{
  "term_label": "cell-cell adhesion",
  "term_id": "GO:0098609",
  "gene_name": "Desmocollin-3",
  "gene": "UniProtKB:Q14574",
  "gene_symbol": "DSC3"
}